{
  "gene_symbol": "ZNF777",
  "term_id": "GO:0000981",
  "gene_name": "Zinc finger protein 777",
  "gene": "UniProtKB:Q9ULD5",
  "term_label": "DNA-binding transcription factor activity, RNA polymerase II-specific"
}